{
  "term_label": "negative regulation of stress fiber assembly",
  "gene": "UniProtKB:A8MT19",
  "gene_symbol": "RHPN2P1",
  "gene_name": "Putative rhophilin-2-like protein RHPN2P1",
  "term_id": "GO:0051497"
}